{
  "term_id": "GO:0043186",
  "term_label": "P granule",
  "gene": "UniProtKB:Q8NHU6",
  "gene_symbol": "TDRD7",
  "gene_name": "Tudor domain-containing protein 7"
}